{
  "term_id": "GO:0000981",
  "gene_symbol": "CEBPB",
  "gene_name": "CCAAT_enhancer-binding protein beta",
  "gene": "UniProtKB:P17676",
  "term_label": "DNA-binding transcription factor activity, RNA polymerase II-specific"
}